{
  "gene_name": "Adipose-secreted signaling protein",
  "gene": "UniProtKB:Q9GZN8",
  "term_label": "Unknown biological process",
  "gene_symbol": "ADISSP",
  "term_id": "UNKNOWN:0002"
}